{
  "gene_name": "Ferric-chelate reductase 1",
  "gene_symbol": "FRRS1",
  "term_label": "intracellular iron ion homeostasis",
  "term_id": "GO:0006879",
  "gene": "UniProtKB:Q6ZNA5"
}